{
  "term_label": "Unknown cellular component",
  "gene_symbol": "AP1S1",
  "gene": "UniProtKB:P61966",
  "gene_name": "AP-1 complex subunit sigma-1A",
  "term_id": "UNKNOWN:0003"
}